G-quadruplex DNA formation [GO:0071919] (biological process) References: PMID:20098422 Sources: GOC:sre Definition: A DNA metabolic process that results in the formation of G-quadruplex DNA structures, in which groups of four guanines adopt a flat, cyclic Hoogsteen hydrogen-bonding arrangement known as a guanine tetrad or G-quartet. The stacking of several layers of G-quartets forms G-quadruplexes, in which one or more DNA single strands are assembled in parallel and/or antiparallel, with interactions that can be either intra- or intermolecular in nature. Also known as: G quadruplex DNA formation, G quartet DNA formation, G-quartet DNA formation Relationships: is a type of DNA metabolic process [GO:0006259]